neuronal stem cell division [GO:0036445] (biological process) Definition: The self-renewing division of a neuronal stem cell. Sources: CL:0000047, GOC:nhn Also known as: NSC division Relationships: is a type of GO:0048103